{
  "gene_name": "T-cell acute lymphocytic leukemia protein 1",
  "gene_symbol": "TAL1",
  "term_label": "DNA-binding transcription factor activity, RNA polymerase II-specific",
  "gene": "UniProtKB:P17542",
  "term_id": "GO:0000981"
}